{
  "term_id": "GO:0000462",
  "gene_symbol": "UTP25",
  "term_label": "maturation of SSU-rRNA from tricistronic rRNA transcript (SSU-rRNA, 5.8S rRNA, LSU-rRNA)",
  "gene_name": "U3 small nucleolar RNA-associated protein 25 homolog",
  "gene": "UniProtKB:Q68CQ4"
}